pentose metabolic process [GO:0019321] (biological process) Subtypes: xylulose metabolic process [GO:0005997], D-ribose metabolic process [GO:0006014], GO:0019322, pentose catabolic process [GO:0019323], L-lyxose metabolic process [GO:0019324], arabinose metabolic process [GO:0019566], D-xylose metabolic process [GO:0042732] Sources: ISBN:0198506732 Relationships: is a type of GO:0005996 Definition: The chemical reactions and pathways involving a pentose, any monosaccharide with a chain of five carbon atoms in the molecule. Also known as: pentose metabolism